{
  "term_id": "GO:0034987",
  "gene_symbol": "IGHG4",
  "gene": "UniProtKB:P01861",
  "gene_name": "Immunoglobulin heavy constant gamma 4",
  "term_label": "immunoglobulin receptor binding"
}